{
  "term_label": "uridine catabolic process",
  "gene": "UniProtKB:Q16831",
  "term_id": "GO:0006218",
  "gene_symbol": "UPP1",
  "gene_name": "Uridine phosphorylase 1"
}